interleukin-1 receptor complex [GO:0045323] (cellular component) Definition: A protein complex that binds interleukin-1; comprises an alpha and a beta subunit. Sources: GOC:mah, InterPro:IPR004075 Relationships: is a type of plasma membrane signaling receptor complex [GO:0098802] Also known as: IL-1 receptor complex